{
  "gene": "UniProtKB:O95644",
  "gene_symbol": "NFATC1",
  "term_label": "nucleus",
  "gene_name": "Nuclear factor of activated T-cells, cytoplasmic 1",
  "term_id": "GO:0005634"
}